{
  "gene_name": "E3 ubiquitin-protein ligase MARCHF6",
  "term_id": "GO:0036503",
  "term_label": "ERAD pathway",
  "gene_symbol": "MARCHF6",
  "gene": "UniProtKB:O60337"
}